{
  "term_id": "UNKNOWN:0002",
  "gene": "UniProtKB:Q9BXT8",
  "gene_symbol": "RNF17",
  "gene_name": "RING finger protein 17",
  "term_label": "Unknown biological process"
}